{
  "gene": "UniProtKB:Q14571",
  "term_label": "release of sequestered calcium ion into cytosol",
  "term_id": "GO:0051209",
  "gene_name": "Inositol 1,4,5-trisphosphate receptor type 2",
  "gene_symbol": "ITPR2"
}